{
  "gene": "UniProtKB:Q99750",
  "term_id": "UNKNOWN:0001",
  "gene_name": "MyoD family inhibitor",
  "term_label": "Unknown molecular function",
  "gene_symbol": "MDFI"
}